{
  "gene": "UniProtKB:Q96J94",
  "gene_symbol": "PIWIL1",
  "term_id": "GO:0031047",
  "term_label": "regulatory ncRNA-mediated gene silencing",
  "gene_name": "Piwi-like protein 1"
}